{
  "gene_name": "PIH1 domain-containing protein 2",
  "term_label": "ribonucleoprotein complex",
  "gene_symbol": "PIH1D2",
  "gene": "UniProtKB:Q8WWB5",
  "term_id": "GO:1990904"
}